calcium ion sequestering activity [GO:0140314] (molecular function) References: PMID:13130076 Relationships: is a type of metal ion sequestering activity [GO:0140487]; has part GO:0005509 Definition: Binding to a calcium ion to prevent it from interacting with other partners or to inhibit its localization to the area of the cell or complex where it is active.